{
  "gene_name": "RNA-binding protein 12",
  "gene_symbol": "RBM12",
  "gene": "UniProtKB:Q9NTZ6",
  "term_id": "GO:1990904",
  "term_label": "ribonucleoprotein complex"
}